sporoplasm [GO:0044100] (cellular component) References: PMID:12076771, PMID:16004371, PMID:9723921 Sources: GOC:mf Definition: The complex infective apparatus corresponding to the central mass of cytoplasm within a spore that is injected into a host cell by various parasitic microorganisms. Relationships: is a type of intracellular anatomical structure [GO:0005622]